{
  "gene_name": "F-box only protein 17",
  "term_label": "ubiquitin protein ligase activity",
  "gene": "UniProtKB:Q96EF6",
  "term_id": "GO:0061630",
  "gene_symbol": "FBXO17"
}